N-acetyl-gamma-aminoadipyl-phosphate reductase activity [GO:0043870] (molecular function) Definition: Catalysis of the reaction: N(2)-acetyl-L-aminoadipate-semialdehyde + NADP+ + phosphate = N(2)-acetyl-L-gamma-aminoadipyl phosphate + NADPH. Sources: RHEA:41948 Also known as: NAGSA dehydrogenase activity, N-acetyl-alpha-glutamyl-phosphate reductase activity, N-acetyl-aminoadipate semialdehyde dehydrogenase activity, AGPR, ArgC, LysY Note: This function is part of the prokaryotic alpha-aminoadipate lysine biosynthesis pathway. Relationships: is a type of oxidoreductase activity, acting on the aldehyde or oxo group of donors, NAD or NADP as acceptor [GO:0016620]